left posteriolateral flagellum [GO:0097556] (cellular component) Definition: A cilium (also called flagellum) found in Giardia species (trophozoite stage). It is nucleated by the left posteriolateral basal body and extends cytoplasmically toward the cell posterior, marking the left anterior boundary of the lateral shield and the left lateral region of the funis before exiting at the left lateral region of the cell body. Also known as: left posteriolateral cilium, left posterolateral cilium, left posterolateral flagellum Relationships: is a type of 9+2 motile cilium [GO:0097729] References: PMID:16607022, PMID:5961344 Sources: GOC:giardia, ISBN:9780124260207 Note: Note that we deem cilium and microtubule-based flagellum to be equivalent; the primary term name reflects frequency of use. Also note that, due to the asymmetric nature of the Giardia trophozoite, this term is defined spatially as the trophozoite is viewed from the dorsal side, with the two nuclei dorsal to the ventral disc, and the ventral disc toward the anterior.